{
  "term_id": "GO:0001650",
  "gene_name": "Ribonuclease P protein subunit p38",
  "gene_symbol": "RPP38",
  "term_label": "fibrillar center",
  "gene": "UniProtKB:P78345"
}